positive regulation of interleukin-17 production [GO:0032740] (biological process) References: PMID:16482511 Sources: GOC:add, GOC:mah Definition: Any process that activates or increases the frequency, rate, or extent of production of any member of the interleukin-17 family of cytokines. Also known as: positive regulation of CTLA-8 production, positive regulation of Cytotoxic T-lymphocyte-associated antigen 8 production, positive regulation of IL-17 production, up regulation of interleukin-17 production, up-regulation of interleukin-17 production, upregulation of interleukin-17 production, activation of interleukin-17 production, positive regulation of interleukin-17 biosynthetic process, positive regulation of interleukin-17 secretion, stimulation of interleukin-17 production Relationships: is a type of positive regulation of cytokine production [GO:0001819]; is a type of regulation of interleukin-17 production [GO:0032660]; positively regulates interleukin-17 production [GO:0032620] Subtypes: GO:0150153